positive regulation of memory T cell differentiation [GO:0043382] (biological process) Sources: ISBN:0781735149 Definition: Any process that activates or increases the frequency, rate or extent of memory T cell differentiation. Also known as: positive regulation of memory T lymphocyte differentiation, positive regulation of memory T-cell differentiation, positive regulation of memory T-lymphocyte differentiation, up regulation of memory T cell differentiation, up-regulation of memory T cell differentiation, upregulation of memory T cell differentiation, activation of memory T cell differentiation, stimulation of memory T cell differentiation, positive regulation of memory T cell development Relationships: is a type of positive regulation of immune effector process [GO:0002699]; is a type of regulation of memory T cell differentiation [GO:0043380]; is a type of positive regulation of T cell differentiation [GO:0045582]; is a type of GO:0050778; positively regulates memory T cell differentiation [GO:0043379] Note: Note that immunologists typically use the word 'development' to refer to cells of B or T cell lineages undergoing the process that GO describes as 'cell differentiation'.